{
  "gene_name": "Na(+)_citrate cotransporter",
  "term_id": "GO:0017153",
  "gene_symbol": "SLC13A5",
  "term_label": "sodium:dicarboxylate symporter activity",
  "gene": "UniProtKB:Q86YT5"
}